{
  "gene": "UniProtKB:Q5SSG8",
  "term_label": "Unknown molecular function",
  "gene_name": "Mucin-21",
  "term_id": "UNKNOWN:0001",
  "gene_symbol": "MUC21"
}